{
  "gene": "UniProtKB:Q86VM9",
  "term_id": "UNKNOWN:0003",
  "term_label": "Unknown cellular component",
  "gene_name": "Zinc finger CCCH domain-containing protein 18",
  "gene_symbol": "ZC3H18"
}